{
  "gene_name": "Zinc finger protein 610",
  "term_id": "GO:0006357",
  "term_label": "regulation of transcription by RNA polymerase II",
  "gene": "UniProtKB:Q8N9Z0",
  "gene_symbol": "ZNF610"
}